regulation of prostaglandin catabolic process [GO:1905828] (biological process) References: PMID:12432938 Sources: GOC:TermGenie, GO_REF:0000058 Also known as: regulation of prostaglandin breakdown, regulation of prostaglandin catabolism, regulation of prostaglandin degradation Subtypes: GO:1905829, positive regulation of prostaglandin catabolic process [GO:1905830] Definition: Any process that modulates the frequency, rate or extent of prostaglandin catabolic process. Relationships: is a type of regulation of lipid catabolic process [GO:0050994]; regulates GO:1905344